{
  "term_label": "Unknown molecular function",
  "gene": "UniProtKB:Q8N8K9",
  "gene_name": "Uncharacterized protein KIAA1958",
  "term_id": "UNKNOWN:0001",
  "gene_symbol": "KIAA1958"
}